{
  "gene": "UniProtKB:P50995",
  "gene_symbol": "ANXA11",
  "term_id": "GO:0005634",
  "term_label": "nucleus",
  "gene_name": "Annexin A11"
}